histone H3K36 trimethyltransferase activity [GO:0140955] (molecular function) Definition: Catalysis of the reaction: L-lysyl36-[histone H3] + 3 S-adenosyl-L-methionine = 3 H+ + N6,N6,N6-trimethyl-L-lysyl36-[histone H3] + 3 S-adenosyl-L-homocysteine. This reaction is the successive addition of three methyl groups to the lysine residue at position 36 of histone H3, producing histone H3K36me3. Sources: RHEA:60324 Also known as: histone H3-K36 trimethylation, histone H3K36 trimethylation, histone H3K36 mono/di/trimethylase activity, histone H3K36 trimethylase activity, histone lysine N-trimethyltransferase activity (H3-K36 specific) Note: Comment: Note that the residue position corresponds to the canonical human H3 histone (UniProtKB:P84243); this residue is conserved across all eukaryotes. Residue 1 is the first residue following removal of the initiating Methionine (Met). Note that each histone is encoded by multiple genes, and sequences may vary across different genes within an organism. Relationships: is a type of GO:0046975